{
  "gene_name": "Probable asparagine--tRNA ligase, mitochondrial",
  "gene": "UniProtKB:Q96I59",
  "term_label": "asparagine-tRNA ligase activity",
  "term_id": "GO:0004816",
  "gene_symbol": "NARS2"
}